{
  "gene": "UniProtKB:Q99932",
  "term_id": "UNKNOWN:0001",
  "term_label": "Unknown molecular function",
  "gene_name": "Sperm-associated antigen 8",
  "gene_symbol": "SPAG8"
}